{
  "term_id": "GO:0005549",
  "gene": "UniProtKB:Q8NGI7",
  "gene_symbol": "OR10V1",
  "gene_name": "Olfactory receptor 10V1",
  "term_label": "odorant binding"
}